{
  "gene": "UniProtKB:Q8IXH8",
  "term_id": "GO:0044331",
  "gene_name": "Cadherin-like protein 26",
  "term_label": "cell-cell adhesion mediated by cadherin",
  "gene_symbol": "CDH26"
}